{
  "term_id": "GO:0007165",
  "gene_name": "Caspase recruitment domain-containing protein 11",
  "term_label": "signal transduction",
  "gene": "UniProtKB:Q9BXL7",
  "gene_symbol": "CARD11"
}